regulation of glomerular mesangial cell proliferation [GO:0072124] (BP) Sources: GOC:mtg_kidney_jan10 Subtypes: negative regulation of glomerular mesangial cell proliferation [GO:0072125], GO:0072126, GO:0072301, regulation of mesonephric glomerular mesangial cell proliferation [GO:2000090] Definition: Any process that modulates the frequency, rate or extent of glomerular mesangial cell proliferation. Relationships: is a type of regulation of cell proliferation involved in kidney development [GO:1901722]; RO_0002211 glomerular mesangial cell proliferation [GO:0072110]